calcium import into the mitochondrion [GO:0036444] (biological process) Definition: A process in which a calcium ion (Ca2+) is transported from the cytosol into the mitochondrial matrix. Sources: GOC:vw Also known as: calcium ion import into mitochondrion, mitochondrial calcium ion import, calcium ion transmembrane import into mitochondrion, mitochondrial calcium uptake Relationships: is a type of mitochondrial calcium ion transmembrane transport [GO:0006851] Subtypes: calcium import into the mitochondrion involved in negative regulation of presynaptic cytosolic calcium concentration [GO:1905743] Regulation: RO_0002211 by regulation of calcium import into the mitochondrion [GO:0110097]; RO_0002213 by positive regulation of calcium import into the mitochondrion [GO:0110098]; negatively regulated by GO:0110099